{
  "gene": "UniProtKB:O94810",
  "gene_name": "Regulator of G-protein signaling 11",
  "gene_symbol": "RGS11",
  "term_id": "GO:0005096",
  "term_label": "GTPase activator activity"
}